N-terminal protein N-methyltransferase activity [GO:0071885] (molecular function) References: PMID:20481588 Relationships: is_a protein methyltransferase activity [GO:0008276]; is_a GO:0008757 Also known as: X-Pro-Lys N-terminal methyltransferase Definition: Catalysis of the transfer of a methyl group from S-adenosyl-L-methionine (AdoMet) to the alpha-amino group of the N-terminal amino or imino acid residue of a protein substrate. For example, yeast Tae1p and mammalian family member METTL11A preferentially modify the N-terminal residue of substrates with the N-terminal sequence X-Pro-Lys, where X can be Pro, Ala, or Ser.